{
  "term_id": "GO:0000981",
  "term_label": "DNA-binding transcription factor activity, RNA polymerase II-specific",
  "gene": "UniProtKB:O15198",
  "gene_symbol": "SMAD9",
  "gene_name": "Mothers against decapentaplegic homolog 9"
}